{
  "gene": "UniProtKB:Q9NSD4",
  "term_id": "GO:0000981",
  "gene_name": "Zinc finger protein 275",
  "gene_symbol": "ZNF275",
  "term_label": "DNA-binding transcription factor activity, RNA polymerase II-specific"
}